{
  "gene_name": "Ret finger protein-like 4A",
  "term_label": "innate immune response",
  "gene_symbol": "RFPL4A",
  "gene": "UniProtKB:A6NLU0",
  "term_id": "GO:0045087"
}